{
  "gene_name": "Putative bifunctional UDP-N-acetylglucosamine transferase and deubiquitinase ALG13",
  "term_label": "Unknown cellular component",
  "gene_symbol": "ALG13",
  "term_id": "UNKNOWN:0003",
  "gene": "UniProtKB:Q9NP73"
}